{
  "term_id": "GO:0005737",
  "gene": "UniProtKB:Q15046",
  "gene_symbol": "KARS1",
  "term_label": "cytoplasm",
  "gene_name": "Lysine--tRNA ligase"
}